{
  "term_id": "GO:0008089",
  "term_label": "anterograde axonal transport",
  "gene_symbol": "ARL8A",
  "gene_name": "ADP-ribosylation factor-like protein 8A",
  "gene": "UniProtKB:Q96BM9"
}